{
  "term_id": "UNKNOWN:0003",
  "term_label": "Unknown cellular component",
  "gene": "UniProtKB:Q96C45",
  "gene_symbol": "ULK4",
  "gene_name": "Serine_threonine-protein kinase ULK4"
}